{
  "gene": "UniProtKB:P51965",
  "term_label": "protein K48-linked ubiquitination",
  "gene_symbol": "UBE2E1",
  "gene_name": "Ubiquitin-conjugating enzyme E2 E1",
  "term_id": "GO:0070936"
}